{
  "term_label": "immune receptor activity",
  "gene_symbol": "LAIR2",
  "gene": "UniProtKB:Q6ISS4",
  "gene_name": "Leukocyte-associated immunoglobulin-like receptor 2",
  "term_id": "GO:0140375"
}